negative regulation of dendritic cell cytokine production [GO:0002731] (biological process) Sources: GOC:add Also known as: down regulation of dendritic cell cytokine production, down-regulation of dendritic cell cytokine production, downregulation of dendritic cell cytokine production, inhibition of dendritic cell cytokine production Definition: Any process that stops, prevents, or reduces the frequency, rate, or extent of dendritic cell cytokine production. Subtypes: negative regulation of myeloid dendritic cell cytokine production [GO:0002734], negative regulation of plasmacytoid dendritic cell cytokine production [GO:0002737] Relationships: is a type of negative regulation of leukocyte mediated immunity [GO:0002704]; is a type of negative regulation of cytokine production involved in immune response [GO:0002719]; is a type of regulation of dendritic cell cytokine production [GO:0002730]; negatively regulates dendritic cell cytokine production [GO:0002371]